{
  "term_id": "GO:0005829",
  "gene": "UniProtKB:Q9NVE5",
  "gene_name": "Ubiquitin carboxyl-terminal hydrolase 40",
  "term_label": "cytosol",
  "gene_symbol": "USP40"
}